{
  "gene": "UniProtKB:Q9BRQ3",
  "term_label": "Unknown biological process",
  "term_id": "UNKNOWN:0002",
  "gene_name": "Uridine diphosphate glucose pyrophosphatase NUDT22",
  "gene_symbol": "NUDT22"
}